{
  "gene": "UniProtKB:Q9BQ51",
  "term_id": "GO:0031295",
  "gene_name": "Programmed cell death 1 ligand 2",
  "term_label": "T cell costimulation",
  "gene_symbol": "PDCD1LG2"
}